{
  "gene_name": "Nucleotide-binding oligomerization domain-containing protein 2",
  "term_label": "defense response to bacterium",
  "term_id": "GO:0042742",
  "gene": "UniProtKB:Q9HC29",
  "gene_symbol": "NOD2"
}